sorbose dehydrogenase activity [GO:0050288] (molecular function) Also known as: L-sorbose:(acceptor) 5-oxidoreductase activity, L-sorbose:acceptor 5-oxidoreductase activity Definition: Catalysis of the reaction: L-sorbose + A = 5-dehydro-D-fructose + AH(2). Relationships: is a type of oxidoreductase activity, acting on CH-OH group of donors [GO:0016614] Sources: EC:1.1.99.12, RHEA:14713